{
  "gene_name": "Thioredoxin domain-containing protein 6",
  "gene": "UniProtKB:Q86XW9",
  "gene_symbol": "NME9",
  "term_label": "Unknown biological process",
  "term_id": "UNKNOWN:0002"
}